{
  "term_id": "GO:0016324",
  "gene": "UniProtKB:P51159",
  "term_label": "apical plasma membrane",
  "gene_symbol": "RAB27A",
  "gene_name": "Ras-related protein Rab-27A"
}